{
  "term_label": "exogenous lipid antigen binding",
  "gene": "UniProtKB:P29017",
  "gene_name": "T-cell surface glycoprotein CD1c",
  "gene_symbol": "CD1C",
  "term_id": "GO:0030884"
}